{
  "gene": "UniProtKB:P51636",
  "term_label": "insulin receptor signaling pathway",
  "term_id": "GO:0008286",
  "gene_name": "Caveolin-2",
  "gene_symbol": "CAV2"
}